{
  "term_id": "GO:0005829",
  "term_label": "cytosol",
  "gene_symbol": "RBM38",
  "gene_name": "RNA-binding protein 38",
  "gene": "UniProtKB:Q9H0Z9"
}